{
  "term_label": "synapse organization",
  "gene_name": "Liprin-alpha-4",
  "gene_symbol": "PPFIA4",
  "term_id": "GO:0050808",
  "gene": "UniProtKB:O75335"
}